regulation of response to furfural [GO:1901442] (biological process) Subtypes: GO:1901443, positive regulation of response to furfural [GO:1901444] Definition: Any process that modulates the frequency, rate or extent of response to furfural. Sources: GOC:TermGenie, GOC:mengo_curators Relationships: is_a GO:0048583; regulates response to furfural [GO:1901426]